{
  "gene_name": "Probable ATP-dependent RNA helicase DDX52",
  "gene_symbol": "DDX52",
  "term_label": "Unknown molecular function",
  "gene": "UniProtKB:Q9Y2R4",
  "term_id": "UNKNOWN:0001"
}